diglucosylglycerate octanoyltransferase activity [GO:0016414] (molecular function) Also known as: O-octanoyltransferase activity Relationships: is a type of O-acyltransferase activity [GO:0008374] Sources: RHEA:56868 Definition: Catalysis of the reaction: (2R)-2-O-[alpha-D-glucopyranosyl-(1->6)-alpha-D-glucopyranosyl]-glycerate + octanoyl-CoA = (2R)-2-O-[6-O-octanoyl-alpha-D-glucopyranosyl-(1->6)-alpha-D-glucopyranosyl]-glycerate + CoA.